{
  "term_id": "UNKNOWN:0001",
  "gene_symbol": "SAMD3",
  "gene_name": "Sterile alpha motif domain-containing protein 3",
  "gene": "UniProtKB:Q8N6K7",
  "term_label": "Unknown molecular function"
}